polyphosphate-mediated signaling [GO:0110094] (biological process) Also known as: polyphosphate signaling Definition: Any process that mediates the transfer of information from one cell to another using polyphosphate as the signal. References: PMID:27519410, PMID:28584190 Sources: GOC:rjd Relationships: is a type of cell-cell signaling [GO:0007267]